{
  "gene_name": "Atrial natriuretic peptide receptor 3",
  "gene": "UniProtKB:P17342",
  "gene_symbol": "NPR3",
  "term_label": "natriuretic peptide receptor activity",
  "term_id": "GO:0016941"
}